negative regulation of T cell mediated cytotoxicity directed against tumor cell target [GO:0002853] (BP) Relationships: is a type of GO:0001915; is a type of negative regulation of T cell mediated immune response to tumor cell [GO:0002841]; is a type of GO:0002852; negatively regulates GO:0002419 Definition: Any process that stops, prevents, or reduces the frequency, rate, or extent of T cell mediated cytotoxicity directed against a tumor cell target. Sources: GOC:add Also known as: down regulation of T cell mediated cytotoxicity directed against tumor cell target, down-regulation of T cell mediated cytotoxicity directed against tumor cell target, downregulation of T cell mediated cytotoxicity directed against tumor cell target, inhibition of T cell mediated cytotoxicity directed against tumor cell target